regulation of hemocyte differentiation [GO:0045610] (biological process) Definition: Any process that modulates the frequency, rate or extent of hemocyte differentiation. Relationships: is a type of regulation of immune system process [GO:0002682]; is a type of GO:0045595; is a type of regulation of multicellular organismal process [GO:0051239]; RO_0002211 hemocyte differentiation [GO:0042386] Subtypes: regulation of lamellocyte differentiation [GO:0035203], regulation of crystal cell differentiation [GO:0042689], negative regulation of hemocyte differentiation [GO:0045611], positive regulation of hemocyte differentiation [GO:0045612], regulation of plasmatocyte differentiation [GO:0045613] Sources: GOC:go_curators Also known as: regulation of arthropod blood cell differentiation